{
  "gene": "UniProtKB:A8K855",
  "term_id": "GO:0098797",
  "term_label": "plasma membrane protein complex",
  "gene_symbol": "EFCAB7",
  "gene_name": "EF-hand calcium-binding domain-containing protein 7"
}